{
  "term_label": "endoplasmic reticulum membrane",
  "gene_symbol": "SGPP2",
  "gene": "UniProtKB:Q8IWX5",
  "term_id": "GO:0005789",
  "gene_name": "Sphingosine-1-phosphate phosphatase 2"
}